phloroglucinol reductase activity [GO:0018510] (molecular function) Relationships: is_a oxidoreductase activity, acting on the CH-CH group of donors, NAD or NADP as acceptor [GO:0016628] Definition: Catalysis of the reaction: dihydrophloroglucinol + NADP+ = H+ + NADPH + phloroglucinol. Also known as: dihydrophloroglucinol:NADP+ oxidoreductase activity Sources: EC:1.3.1.57, RHEA:10080